{
  "gene_symbol": "NBPF11",
  "gene": "UniProtKB:Q86T75",
  "term_label": "Unknown biological process",
  "gene_name": "Neuroblastoma breakpoint family member 11",
  "term_id": "UNKNOWN:0002"
}